{
  "gene_symbol": "MEGF11",
  "term_label": "substrate adhesion-dependent cell spreading",
  "gene": "UniProtKB:A6BM72",
  "gene_name": "Multiple epidermal growth factor-like domains protein 11",
  "term_id": "GO:0034446"
}